{
  "term_id": "GO:0035267",
  "gene_symbol": "ACTL6B",
  "gene": "UniProtKB:O94805",
  "term_label": "NuA4 histone acetyltransferase complex",
  "gene_name": "Actin-like protein 6B"
}